negative regulation of formation of radial glial scaffolds [GO:0061925] (BP) References: PMID:22076441 Also known as: negative regulation of radial glial scaffold formation, negative regulation of Bergmann fiber biosynthesis, negative regulation of Bergmann fiber formation Definition: Any process that reduces the frequency, rate or extent of the formation of radial glial scaffolds. The scaffolds are used as a substrate for the radial migration of cells. Relationships: is a type of negative regulation of cell morphogenesis [GO:0010771]; is a type of regulation of formation of radial glial scaffolds [GO:0061924]; negatively regulates formation of radial glial scaffolds [GO:0021943]